{
  "gene_name": "Protein Wnt-3a",
  "gene": "UniProtKB:P56704",
  "term_id": "GO:0030182",
  "term_label": "neuron differentiation",
  "gene_symbol": "WNT3A"
}